{
  "gene": "UniProtKB:Q8NC67",
  "term_label": "regulation of neurotransmitter receptor localization to postsynaptic specialization membrane",
  "gene_name": "Neuropilin and tolloid-like protein 2",
  "term_id": "GO:0098696",
  "gene_symbol": "NETO2"
}